{
  "gene_symbol": "CSNK1D",
  "gene_name": "Casein kinase I isoform delta",
  "term_label": "positive regulation of proteasomal ubiquitin-dependent protein catabolic process",
  "term_id": "GO:0032436",
  "gene": "UniProtKB:P48730"
}